{
  "gene_symbol": "USP17L12",
  "gene_name": "Ubiquitin carboxyl-terminal hydrolase 17-like protein 12",
  "term_id": "GO:0004843",
  "term_label": "cysteine-type deubiquitinase activity",
  "gene": "UniProtKB:C9JPN9"
}